{
  "gene_symbol": "CIMAP3",
  "term_id": "GO:0008092",
  "gene": "UniProtKB:Q8TCI5",
  "term_label": "cytoskeletal protein binding",
  "gene_name": "Protein pitchfork"
}